{
  "gene_name": "Keratin, type I cytoskeletal 14",
  "gene_symbol": "KRT14",
  "term_label": "intermediate filament organization",
  "gene": "UniProtKB:P02533",
  "term_id": "GO:0045109"
}